{
  "gene": "UniProtKB:Q7Z5L3",
  "gene_symbol": "C1QL2",
  "term_id": "GO:0043083",
  "term_label": "synaptic cleft",
  "gene_name": "Complement C1q-like protein 2"
}